sphingomyelin transfer activity [GO:0140338] (molecular function) Relationships: is a type of phospholipid transfer activity [GO:0120014]; is a type of GO:0120016 Also known as: sphingosine transmembrane transporter activity, sphingomyelin carrier activity Definition: Removes a sphingomyelin from the outer leaflet of a donor membrane, transports it through the aqueous phase while protected in a hydrophobic pocket, and brings it to the outer leaflet of an acceptor membrane. References: PMID:9132017